{
  "gene_name": "DDB1- and CUL4-associated factor 13",
  "gene_symbol": "DCAF13",
  "term_label": "nucleolus",
  "gene": "UniProtKB:Q9NV06",
  "term_id": "GO:0005730"
}